response to inactivity [GO:0014854] (biological process) Definition: Any process that results in a change in state or activity of a cell or an organism (in terms of movement, secretion, enzyme production, gene expression, etc.) as a result of an inactivity stimulus. Subtypes: detection of inactivity [GO:0014863], response to muscle inactivity [GO:0014870] Sources: GOC:mtg_muscle Relationships: is a type of GO:0050896